dethiobiotin binding [GO:1901602] (molecular function) Definition: Binding to dethiobiotin. Sources: GOC:TermGenie Relationships: is a type of amide binding [GO:0033218]; is a type of monocarboxylic acid binding [GO:0033293]; is a type of heterocyclic compound binding [GO:1901363]